{
  "gene": "UniProtKB:Q9H4I9",
  "term_id": "GO:0036444",
  "gene_symbol": "SMDT1",
  "term_label": "calcium import into the mitochondrion",
  "gene_name": "Essential MCU regulator, mitochondrial"
}